{
  "gene": "UniProtKB:Q2TV78",
  "term_label": "extracellular space",
  "gene_name": "Putative macrophage stimulating 1-like protein",
  "gene_symbol": "MST1L",
  "term_id": "GO:0005615"
}